citrate transport [GO:0015746] (biological process) Definition: The directed movement of citrate, 2-hydroxy-1,2,3-propanetricarboxylate, into, out of or within a cell, or between cells, by means of some agent such as a transporter or pore. Subtypes: GO:0006843, GO:0046720 Relationships: is a type of tricarboxylic acid transport [GO:0006842] Sources: GOC:krc